{
  "term_id": "UNKNOWN:0003",
  "gene_name": "Kelch domain-containing protein 8A",
  "term_label": "Unknown cellular component",
  "gene": "UniProtKB:Q8IYD2",
  "gene_symbol": "KLHDC8A"
}